{
  "term_label": "RNA polymerase II cis-regulatory region sequence-specific DNA binding",
  "gene_name": "Zinc finger and BTB domain-containing protein 17",
  "gene": "UniProtKB:Q13105",
  "term_id": "GO:0000978",
  "gene_symbol": "ZBTB17"
}